{
  "term_id": "GO:0015854",
  "gene": "UniProtKB:Q14542",
  "term_label": "guanine transport",
  "gene_symbol": "SLC29A2",
  "gene_name": "Equilibrative nucleoside transporter 2"
}